regulation of neurotransmitter loading into synaptic vesicle [GO:0099162] (BP) Definition: Any process that modulates the frequency, rate or extent of neurotransmitter loading into synaptic vesicles. Relationships: is a type of regulation of neurotransmitter transport [GO:0051588]; is a type of regulation of synaptic vesicle cycle [GO:0098693]; regulates neurotransmitter loading into synaptic vesicle [GO:0098700] References: PMID:25176177 Sources: GOC:dos Also known as: regulation of neurotransmitter uptake into synaptic vesicle, regulation of synaptic vesicle neurotransmitter loading